{
  "gene": "UniProtKB:P48723",
  "term_label": "heat shock protein binding",
  "gene_symbol": "HSPA13",
  "term_id": "GO:0031072",
  "gene_name": "Heat shock 70 kDa protein 13"
}